{
  "term_id": "GO:0001540",
  "term_label": "amyloid-beta binding",
  "gene": "UniProtKB:Q92870",
  "gene_name": "Amyloid beta precursor protein binding family B member 2",
  "gene_symbol": "APBB2"
}